postsynaptic signal transduction [GO:0098926] (biological process) Definition: Signal transduction in which the initial step occurs in a postsynapse. Relationships: is a type of signal transduction [GO:0007165]; is part of GO:0099536 Sources: GOC:dos Also known as: postsynaptic signaling pathway Subtypes: GO:0095500, postsynapse to nucleus signaling pathway [GO:0099527]